negative regulation of complement activation, classical pathway [GO:0045959] (BP) Sources: GOC:go_curators Definition: Any process that stops, prevents, or reduces the frequency, rate or extent of complement activation by the classical pathway. Also known as: down regulation of complement activation, classical pathway, down-regulation of complement activation, classical pathway, downregulation of complement activation, classical pathway, negative regulation of complement cascade, classical pathway, inhibition of complement activation, classical pathway Relationships: is a type of negative regulation of humoral immune response mediated by circulating immunoglobulin [GO:0002924]; is_a regulation of complement activation, classical pathway [GO:0030450]; is a type of negative regulation of complement activation [GO:0045916]; negatively regulates complement activation, classical pathway [GO:0006958]